{
  "term_label": "transcription initiation at RNA polymerase II promoter",
  "term_id": "GO:0006367",
  "gene_name": "General transcription factor IIE subunit 1",
  "gene": "UniProtKB:P29083",
  "gene_symbol": "GTF2E1"
}